{
  "gene_symbol": "PLEKHB1",
  "term_id": "GO:0045595",
  "gene": "UniProtKB:Q9UF11",
  "term_label": "regulation of cell differentiation",
  "gene_name": "Pleckstrin homology domain-containing family B member 1"
}